phytochelatin-metal-sulfur complex formation [GO:0090424] (biological process) Also known as: HWM phytochelatin complex formation, high molecular weight phytochelatin complex formation Sources: GOC:tb Definition: A phytochelatin metabolic process in which a metal and exogenous sulfur are incorporated with phytochelatin to form a complex. Relationships: is a type of phytochelatin metabolic process [GO:0046937]